tRNA re-export from nucleus [GO:0071528] (biological process) Relationships: is a type of tRNA export from nucleus [GO:0006409] Also known as: tRNA reexport from nucleus References: PMID:17475781, PMID:20032305 Sources: GOC:mcc Definition: The directed movement from the nucleus to the cytoplasm of a tRNA that was previously exported to the cytoplasm and then imported back into the nucleus. The processes of primary tRNA export and secondary export (re-export) can be distinguished because in organisms in which tRNA splicing occurs in the cytoplasm, the export of a mature tRNA must occur by re-export.